{
  "gene": "UniProtKB:P01031",
  "gene_name": "Complement C5",
  "gene_symbol": "C5",
  "term_id": "UNKNOWN:0002",
  "term_label": "Unknown biological process"
}